IgX immunoglobulin complex [GO:0071759] (cellular component) Note: Note that an IgX immunoglobulin complex has the function of antigen binding if a suitable antigen is available. Note that IgX is found in amphibians. Definition: A protein complex composed of two identical immunoglobulin heavy chains of the IgX isotype and two identical immunoglobulin light chains, held together by disulfide bonds. An IgX immunoglobulin complex may be embedded in the plasma membrane or present in the extracellular space, in mucosal areas or other tissues, or circulating in the blood or lymph. Relationships: is_a immunoglobulin complex [GO:0019814] Sources: GOC:add, ISBN:0781765196